dihydroceramide fatty acyl 2-hydroxylase activity [GO:0102771] (molecular function) Definition: Catalysis of the reaction: an N-(1,2-saturated acyl)sphinganine + 2 Fe(II)-[cytochrome b5] + 2 H+ + O2 = an N-[(2'R)-hydroxyacyl]sphinganine + 2 Fe(III)-[cytochrome b5] + H2O. Sources: RHEA:46512 Relationships: is a type of GO:0080132 Also known as: plant sphingolipid fatty acid 2-hydroxylase actitivy, sphingolipid very long chain fatty acid alpha-hydroxylase activity